{
  "term_label": "single-stranded DNA binding",
  "gene_symbol": "CTC1",
  "gene": "UniProtKB:Q2NKJ3",
  "gene_name": "CST complex subunit CTC1",
  "term_id": "GO:0003697"
}